cellular response to cyclosporin A [GO:1905238] (biological process) Also known as: cellular response to cyclophilin Relationships: is a type of cellular response to nitrogen compound [GO:1901699]; is a type of cellular response to oxygen-containing compound [GO:1901701]; is a type of response to cyclosporin A [GO:1905237] Definition: Any process that results in a change in state or activity of a cell (in terms of movement, secretion, enzyme production, gene expression, etc.) as a result of a cyclosporin A stimulus. References: PMID:24914722 Sources: GOC:TermGenie, GO_REF:0000071